{
  "term_label": "pexophagy",
  "term_id": "GO:0000425",
  "gene": "UniProtKB:Q5MNZ9",
  "gene_symbol": "WIPI1",
  "gene_name": "WD repeat domain phosphoinositide-interacting protein 1"
}